{
  "gene_symbol": "DLGAP5",
  "term_id": "GO:0051382",
  "gene": "UniProtKB:Q15398",
  "gene_name": "Disks large-associated protein 5",
  "term_label": "kinetochore assembly"
}